{
  "gene": "UniProtKB:Q8IYY4",
  "gene_symbol": "DZIP1L",
  "gene_name": "Cilium assembly protein DZIP1L",
  "term_label": "cytoplasm",
  "term_id": "GO:0005737"
}